cartilage condensation [GO:0001502] (biological process) Definition: The condensation of mesenchymal cells that have been committed to differentiate into chondrocytes. Sources: ISBN:0878932437 Relationships: is a type of cell aggregation [GO:0098743]; is part of skeletal system morphogenesis [GO:0048705]; is part of cartilage development [GO:0051216] Regulation: regulated by regulation of cartilage condensation [GO:1902026]; positively regulated by GO:1902027; negatively regulated by negative regulation of cartilage condensation [GO:1904932]